intestine smooth muscle contraction [GO:0014827] (BP) Sources: GOC:mtg_muscle, MA:0001539, MSH:D007422 Definition: A process in which force is generated within smooth muscle tissue, resulting in a change in muscle geometry. This process occurs in the intestine. Force generation involves a chemo-mechanical energy conversion step that is carried out by the actin/myosin complex activity, which generates force through ATP hydrolysis. The intestine is the section of the alimentary canal from the stomach to the anal canal. It includes the large intestine and small intestine. Relationships: is a type of phasic smooth muscle contraction [GO:0014821]; is a type of gastro-intestinal system smooth muscle contraction [GO:0014831]